indoleamine 2,3-dioxygenase activity [GO:0033754] (molecular function) Sources: RHEA:14189 Relationships: is a type of GO:0016702 Definition: Catalysis of the reaction: D-tryptophan + O2 = N-formyl-D-kynurenine. Also known as: tryptophan pyrrolase activity, D-tryptophan:oxygen 2,3-oxidoreductase (decyclizing) activity, IDO